NAD DNA ADP-ribosyltransferase activity [GO:0140294] (molecular function) Definition: Catalysis of the transfer of the ADP-ribose group of NAD+ to a residue in double-stranded DNA. Subtypes: GO:0030591 References: PMID:27471034, PMID:29361132, PMID:29520010 Relationships: is a type of pentosyltransferase activity [GO:0016763]